positive regulation of establishment of Sertoli cell barrier [GO:1904446] (biological process) Also known as: positive regulation of establishment of BTB, positive regulation of establishment of SCB, positive regulation of establishment of blood-testis barrier, up regulation of establishment of BTB, up regulation of establishment of SCB, up regulation of establishment of Sertoli cell barrier, up regulation of establishment of blood-testis barrier, up-regulation of establishment of BTB, up-regulation of establishment of SCB, up-regulation of establishment of Sertoli cell barrier, up-regulation of establishment of blood-testis barrier, upregulation of establishment of BTB, upregulation of establishment of SCB, upregulation of establishment of Sertoli cell barrier, upregulation of establishment of blood-testis barrier, activation of establishment of BTB, activation of establishment of SCB, activation of establishment of Sertoli cell barrier, activation of establishment of blood-testis barrier Definition: Any process that activates or increases the frequency, rate or extent of establishment of Sertoli cell barrier. References: PMID:18057314 Sources: GOC:TermGenie, GO_REF:0000058 Relationships: is_a positive regulation of cell development [GO:0010720]; is_a regulation of establishment of Sertoli cell barrier [GO:1904444]; is a type of positive regulation of reproductive process [GO:2000243]; positively regulates establishment of Sertoli cell barrier [GO:0097368]